{
  "gene": "UniProtKB:P51843",
  "term_label": "adrenal gland development",
  "term_id": "GO:0030325",
  "gene_symbol": "NR0B1",
  "gene_name": "Nuclear receptor subfamily 0 group B member 1"
}